Tat protein binding [GO:0030957] (molecular function) Relationships: is a type of GO:0061629 Definition: Binding to Tat, a viral transactivating regulatory protein from the human immunodeficiency virus, or the equivalent protein from another virus. References: PMID:9094689 Sources: GOC:mah